{
  "term_id": "GO:0140297",
  "gene_name": "C-terminal-binding protein 2",
  "gene_symbol": "CTBP2",
  "gene": "UniProtKB:P56545",
  "term_label": "DNA-binding transcription factor binding"
}